{
  "term_id": "GO:1902600",
  "gene": "UniProtKB:Q7RTS6",
  "term_label": "proton transmembrane transport",
  "gene_name": "Proton channel OTOP2",
  "gene_symbol": "OTOP2"
}